sterol homeostasis [GO:0055092] (biological process) Subtypes: cholesterol homeostasis [GO:0042632] Sources: GOC:BHF, GOC:rl Definition: Any process involved in the maintenance of an internal steady state of sterol within an organism or cell. Relationships: is a type of lipid homeostasis [GO:0055088]